{
  "term_id": "GO:0001501",
  "gene_symbol": "PAX1",
  "gene_name": "Paired box protein Pax-1",
  "term_label": "skeletal system development",
  "gene": "UniProtKB:P15863"
}